ornithine cyclodeaminase activity [GO:0008473] (molecular function) Sources: EC:4.3.1.12, RHEA:24368 Relationships: is a type of GO:0016841 Definition: Catalysis of the reaction: L-ornithine = L-proline + NH4. Note: Note that cyclodeaminases are lyases according to EC, whereas deaminases are hydrolases. Also known as: L-ornithine ammonia-lyase (cyclizing), L-ornithine ammonia-lyase (cyclizing; L-proline-forming), OCD activity, ornithine cyclase (deaminating) activity, ornithine cyclase activity